{
  "term_id": "GO:0050431",
  "gene_name": "TGF-beta receptor type-2",
  "gene": "UniProtKB:P37173",
  "term_label": "transforming growth factor beta binding",
  "gene_symbol": "TGFBR2"
}